negative regulation of phospholipid efflux [GO:1902999] (BP) Relationships: is a type of regulation of phospholipid efflux [GO:1902994]; is a type of negative regulation of phospholipid transport [GO:2001139]; negatively regulates GO:0033700 References: PMID:12042316 Sources: GOC:TermGenie, GOC:sjp, GO_REF:0000058 Also known as: down regulation of phospholipid efflux, down regulation of phospholipid export, down-regulation of phospholipid efflux, down-regulation of phospholipid export, downregulation of phospholipid efflux, downregulation of phospholipid export, negative regulation of phospholipid export, inhibition of phospholipid efflux, inhibition of phospholipid export Definition: Any process that stops, prevents or reduces the frequency, rate or extent of phospholipid efflux.